alpha-1,4-mannosyltransferase activity [GO:0051751] (molecular function) References: PMID:15772281 Definition: Catalysis of the transfer of a mannose residue to an oligosaccharide, forming an alpha-(1->4) linkage. Subtypes: dol-P-Man:GlcN-acyl-PI alpha-1,4-mannosyltransferase activity [GO:0180041] Relationships: is a type of GO:0000030